{
  "term_id": "GO:0030948",
  "term_label": "negative regulation of vascular endothelial growth factor receptor signaling pathway",
  "gene_symbol": "MMRN2",
  "gene_name": "Multimerin-2",
  "gene": "UniProtKB:Q9H8L6"
}